positive regulation of smooth muscle contraction involved in micturition [GO:1904320] (BP) Definition: Any process that activates or increases the frequency, rate or extent of smooth muscle contraction involved in micturition. Also known as: up regulation of smooth muscle contraction involved in micturition, up-regulation of smooth muscle contraction involved in micturition, upregulation of smooth muscle contraction involved in micturition, activation of smooth muscle contraction involved in micturition, activation of smooth muscle contraction involved in urination, activation of urinary bladder smooth muscle contraction involved in micturition, positive regulation of smooth muscle contraction involved in urination, positive regulation of urinary bladder smooth muscle contraction involved in micturition, up regulation of smooth muscle contraction involved in urination, up regulation of urinary bladder smooth muscle contraction involved in micturition, up-regulation of smooth muscle contraction involved in urination, up-regulation of urinary bladder smooth muscle contraction involved in micturition, upregulation of smooth muscle contraction involved in urination, upregulation of urinary bladder smooth muscle contraction involved in micturition References: PMID:18562635 Sources: GOC:TermGenie, GO_REF:0000058 Relationships: is a type of positive regulation of smooth muscle contraction [GO:0045987]; is a type of regulation of smooth muscle contraction involved in micturition [GO:1904318]; positively regulates GO:0060083